{
  "gene_name": "Transmembrane protein 43",
  "term_id": "GO:0005637",
  "term_label": "nuclear inner membrane",
  "gene": "UniProtKB:Q9BTV4",
  "gene_symbol": "TMEM43"
}